negative regulation of erythrocyte apoptotic process [GO:1902251] (biological process) Relationships: is a type of GO:0033033; is a type of regulation of erythrocyte apoptotic process [GO:1902250]; negatively regulates GO:1902217 Also known as: down regulation of RBC apoptotic process, down regulation of erythrocyte apoptotic process, down regulation of red blood cell apoptotic process, down-regulation of RBC apoptotic process, down-regulation of erythrocyte apoptotic process, down-regulation of red blood cell apoptotic process, downregulation of RBC apoptotic process, downregulation of erythrocyte apoptotic process, downregulation of red blood cell apoptotic process, negative regulation of RBC apoptotic process, negative regulation of red blood cell apoptotic process, down regulation of RBC apoptosis, down regulation of erythrocyte apoptosis, down regulation of red blood cell apoptosis, down-regulation of RBC apoptosis, down-regulation of erythrocyte apoptosis, down-regulation of red blood cell apoptosis, downregulation of RBC apoptosis, downregulation of erythrocyte apoptosis, downregulation of red blood cell apoptosis, inhibition of RBC apoptosis, inhibition of RBC apoptotic process, inhibition of erythrocyte apoptosis, inhibition of erythrocyte apoptotic process, inhibition of red blood cell apoptosis, inhibition of red blood cell apoptotic process, negative regulation of RBC apoptosis, negative regulation of erythrocyte apoptosis, negative regulation of red blood cell apoptosis Definition: Any process that stops, prevents or reduces the frequency, rate or extent of erythrocyte apoptotic process. References: PMID:14569084 Sources: GOC:BHF, GOC:TermGenie, GOC:mtg_apoptosis, GOC:rl